positive regulation of FtsZ-dependent cytokinesis [GO:2000246] (biological process) Definition: Any process that activates or increases the frequency, rate or extent of Ftsz-dependent cytokinesis. Sources: GOC:mah Also known as: positive regulation of prokaryote-type cytokinesis, positive regulation of prokaryotic fission Relationships: is a type of positive regulation of cytokinesis [GO:0032467]; is a type of GO:2000243; is a type of GO:2000244; positively regulates GO:0043093